{
  "gene_name": "Desmocollin-3",
  "term_label": "desmosome",
  "gene": "UniProtKB:Q14574",
  "term_id": "GO:0030057",
  "gene_symbol": "DSC3"
}